{
  "gene_symbol": "SLC2A2",
  "gene": "UniProtKB:P11168",
  "term_id": "GO:0005903",
  "gene_name": "Solute carrier family 2, facilitated glucose transporter member 2",
  "term_label": "brush border"
}